{
  "gene_name": "NADH-cytochrome b5 reductase 1",
  "term_label": "FAD binding",
  "term_id": "GO:0071949",
  "gene_symbol": "CYB5R1",
  "gene": "UniProtKB:Q9UHQ9"
}